{
  "term_label": "mitotic cell cycle",
  "gene_name": "Centromere protein F",
  "term_id": "GO:0000278",
  "gene_symbol": "CENPF",
  "gene": "UniProtKB:P49454"
}